{
  "term_id": "GO:0016929",
  "gene": "UniProtKB:Q96HI0",
  "term_label": "deSUMOylase activity",
  "gene_symbol": "SENP5",
  "gene_name": "Sentrin-specific protease 5"
}